{
  "gene_name": "Phosphatase and actin regulator 1",
  "term_label": "cell motility",
  "gene_symbol": "PHACTR1",
  "gene": "UniProtKB:Q9C0D0",
  "term_id": "GO:0048870"
}